4-methoxybenzoate monooxygenase (O-demethylating) activity [GO:0018690] (molecular function) Also known as: 4-methoxybenzoate monooxygenase activity, 4-methoxybenzoate 4-monooxygenase (O-demethylating), 4-methoxybenzoate O-demethylase activity, 4-methoxybenzoate,hydrogen-donor:oxygen oxidoreductase (O-demethylating), p-anisic O-demethylase activity, piperonylate-4-O-demethylase activity Relationships: is a type of monooxygenase activity [GO:0004497]; is a type of oxidoreductase activity, acting on paired donors, with incorporation or reduction of molecular oxygen [GO:0016705] Sources: EC:1.14.99.15, RHEA:18613 Definition: Catalysis of the reaction: 4-methoxybenzoate + AH(2) + O2 = 4-hydroxybenzoate + A + formaldehyde + H2O.